{
  "term_id": "GO:0016020",
  "term_label": "membrane",
  "gene_name": "Inositol polyphosphate 5-phosphatase OCRL",
  "gene_symbol": "OCRL",
  "gene": "UniProtKB:Q01968"
}